{
  "term_label": "protein-containing complex",
  "term_id": "GO:0032991",
  "gene_name": "Oocyte-expressed protein homolog",
  "gene": "UniProtKB:A6NGQ2",
  "gene_symbol": "OOEP"
}